{
  "term_label": "otolith morphogenesis",
  "gene_symbol": "TTC39C",
  "term_id": "GO:0032474",
  "gene": "UniProtKB:Q8N584",
  "gene_name": "Tetratricopeptide repeat protein 39C"
}